{
  "term_id": "GO:0007507",
  "gene_symbol": "PDLIM7",
  "term_label": "heart development",
  "gene_name": "PDZ and LIM domain protein 7",
  "gene": "UniProtKB:Q9NR12"
}